{
  "term_id": "GO:0005874",
  "gene": "UniProtKB:P59282",
  "term_label": "microtubule",
  "gene_name": "Tubulin polymerization-promoting protein family member 2",
  "gene_symbol": "TPPP2"
}